regulation of macrophage chemotaxis [GO:0010758] (biological process) Subtypes: positive regulation of macrophage chemotaxis [GO:0010759], negative regulation of macrophage chemotaxis [GO:0010760] Sources: GOC:BHF, GOC:dph, GOC:tb Definition: Any process that modulates the rate, frequency or extent of macrophage chemotaxis. Macrophage chemotaxis is the movement of a macrophage in response to an external stimulus. Relationships: is a type of regulation of leukocyte chemotaxis [GO:0002688]; is a type of regulation of macrophage migration [GO:1905521]; regulates macrophage chemotaxis [GO:0048246]